{
  "gene_name": "Ephrin-A5",
  "gene": "UniProtKB:P52803",
  "term_label": "ephrin receptor binding",
  "term_id": "GO:0046875",
  "gene_symbol": "EFNA5"
}